positive regulation of striated muscle tissue development [GO:0045844] (biological process) Relationships: is a type of GO:0016202; is a type of positive regulation of muscle organ development [GO:0048636]; is a type of positive regulation of muscle tissue development [GO:1901863]; positively regulates striated muscle tissue development [GO:0014706] Also known as: up regulation of striated muscle development, up-regulation of striated muscle development, upregulation of striated muscle development, activation of striated muscle development, stimulation of striated muscle development Sources: GOC:go_curators Definition: Any process that activates or increases the frequency, rate or extent of striated muscle development. Subtypes: positive regulation of skeletal muscle tissue development [GO:0048643], positive regulation of cardiac muscle tissue development [GO:0055025]